phosphosulfolactate synthase activity [GO:0043817] (molecular function) Also known as: (2R)-O-phospho-3-sulfolactate sulfo-lyase activity, (2R)-O-phospho-3-sulfolactate sulfo-lyase (phosphoenolpyruvate-forming), (2R)-phospho-3-sulfolactate synthase activity, PSL synthase activity Definition: Catalysis of the reaction: (2R)-O-phospho-3-sulfolactate = phosphoenolpyruvate + sulfite. Relationships: is a type of carbon-sulfur lyase activity [GO:0016846] Sources: EC:4.4.1.19, RHEA:22784